axon extension [GO:0048675] (BP) Regulation: regulated by regulation of axon extension [GO:0030516]; negatively regulated by negative regulation of axon extension [GO:0030517]; positively regulated by positive regulation of axon extension [GO:0045773] Definition: Long distance growth of a single axon process involved in cellular development. Relationships: is a type of neuron projection extension [GO:1990138]; is part of axonogenesis [GO:0007409] Sources: GOC:BHF, GOC:dgh, GOC:dph, GOC:jid, GOC:lm Also known as: axon extension involved in development Subtypes: axon extension involved in regeneration [GO:0048677], axon extension involved in axon guidance [GO:0048846]